phosphotransferase activity, carboxyl group as acceptor [GO:0016774] (molecular function) Sources: EC:2.7.2.- Subtypes: acetylglutamate kinase activity [GO:0003991], aspartate kinase activity [GO:0004072], GO:0004349, GO:0004618, acetate kinase activity [GO:0008776], carbamate kinase activity [GO:0008804], propionate kinase activity [GO:0008980], N2-acetyl-L-aminoadipate kinase activity [GO:0043744], acetate kinase (diphosphate) activity [GO:0047601], GO:0047758, butyrate kinase activity [GO:0047761], formate kinase activity [GO:0047900], GO:0050191 Definition: Catalysis of the transfer of a phosphorus-containing group from one compound (donor) to a carboxyl group (acceptor). Relationships: is a type of transferase activity, transferring phosphorus-containing groups [GO:0016772]